regulation of glomerulus development [GO:0090192] (biological process) Definition: Any process that modulates the rate, frequency or extent of glomerulus development, the progression of the glomerulus over time from its initial formation until its mature state. The glomerulus is a capillary tuft surrounded by Bowman's capsule in nephrons of the vertebrate kidney. Relationships: is a type of regulation of kidney development [GO:0090183]; RO_0002211 glomerulus development [GO:0032835] Sources: GOC:dph, GOC:tb, GOC:yaf Subtypes: regulation of metanephric glomerulus development [GO:0072298], GO:0090193, negative regulation of glomerulus development [GO:0090194], regulation of mesonephric glomerulus development [GO:2000087]